{
  "gene_name": "Sodium_hydrogen exchanger 11",
  "term_id": "GO:0098719",
  "term_label": "sodium ion import across plasma membrane",
  "gene_symbol": "SLC9C2",
  "gene": "UniProtKB:Q5TAH2"
}